{
  "term_id": "GO:0005634",
  "gene_symbol": "FUBP3",
  "gene_name": "Far upstream element-binding protein 3",
  "gene": "UniProtKB:Q96I24",
  "term_label": "nucleus"
}